{
  "term_id": "GO:0045109",
  "gene_name": "Keratin, type I cytoskeletal 10",
  "term_label": "intermediate filament organization",
  "gene_symbol": "KRT10",
  "gene": "UniProtKB:P13645"
}